Bcl3/NF-kappaB2 complex [GO:0033257] (cellular component) Definition: A protein complex containing one Bcl protein and one or more copies of NF-kappaB2; formation of complexes of different stoichiometry depends on the Bcl3:NF-kappaB2 ratio, and allow Bcl3 to exert different regulatory effects on NF-kappaB2-dependent transcription. Relationships: is a type of I-kappaB/NF-kappaB complex [GO:0033256] References: PMID:9407099 Sources: GOC:mah Also known as: Bcl3-p52 complex, Bcl3-NFKB2 complex